{
  "term_label": "olfactory receptor activity",
  "gene_symbol": "OR5BS1",
  "gene_name": "Olfactory receptor",
  "term_id": "GO:0004984",
  "gene": "UniProtKB:A0A2R8YED5"
}